{
  "gene_symbol": "ZNF383",
  "term_id": "UNKNOWN:0003",
  "gene_name": "Zinc finger protein 383",
  "gene": "UniProtKB:Q8NA42",
  "term_label": "Unknown cellular component"
}